{
  "gene": "UniProtKB:Q9UIL4",
  "term_id": "GO:0016887",
  "term_label": "ATP hydrolysis activity",
  "gene_name": "Kinesin-like protein KIF25",
  "gene_symbol": "KIF25"
}